{
  "gene_name": "Collagen alpha-2(V) chain",
  "term_id": "GO:0005588",
  "term_label": "collagen type V trimer",
  "gene": "UniProtKB:P05997",
  "gene_symbol": "COL5A2"
}